{
  "term_label": "alpha-N-acetylgalactosaminide alpha-2,6-sialyltransferase activity",
  "gene": "UniProtKB:Q9UJ37",
  "gene_symbol": "ST6GALNAC2",
  "term_id": "GO:0001665",
  "gene_name": "Alpha-N-acetylgalactosaminide alpha-2,6-sialyltransferase 2"
}